cell adhesion receptor activity [GO:0004895] (molecular function) Sources: GOC:BHF-UCL, Wikipedia:Cell_adhesion Note: Reinstated term from obsolete. Definition: The binding by a cell-adhesion protein on the cell surface to an extracellular matrix component, to mediate adhesion of the cell to the external substrate or to another cell and to initiate intracellular signaling. Cell adhesion receptors include integrins and cadherins. Relationships: is a type of signaling receptor activity [GO:0038023]; is_a cell adhesion mediator activity [GO:0098631]